{
  "gene": "UniProtKB:Q7RTR0",
  "term_id": "GO:0005737",
  "gene_name": "NACHT, LRR and PYD domains-containing protein 9",
  "term_label": "cytoplasm",
  "gene_symbol": "NLRP9"
}